{
  "gene": "UniProtKB:P20231",
  "term_label": "extracellular space",
  "gene_symbol": "TPSB2",
  "gene_name": "Tryptase beta-2",
  "term_id": "GO:0005615"
}